phosphoribosylformylglycinamidine synthase activity [GO:0004642] (molecular function) Sources: EC:6.3.5.3, RHEA:17129 Definition: Catalysis of the reaction: N(2)-formyl-N(1)-(5-phospho-D-ribosyl)glycinamide + L-glutamine + ATP + H2O = 2-(formamido)-N(1)-(5-phospho-D-ribosyl)acetamidine + L-glutamate + ADP + 2 H+ + phosphate. Also known as: 2-N-formyl-1-N-(5-phospho-D-ribosyl)glycinamide:L-glutamine amido-ligase (ADP-forming), 5'-phosphoribosylformylglycinamide:L-glutamine amido-ligase (ADP-forming), FGAM synthase activity, FGAM synthetase activity, FGAR amidotransferase activity, FGARAT activity, N2-formyl-N1-(5-phospho-D-ribosyl)glycinamide:L-glutamine amido-ligase (ADP-forming), formylglycinamide ribonucloetide amidotransferase activity, formylglycinamide ribotide amidotransferase activity, phosphoribosylformylglycinamidine synthetase activity, phosphoribosylformylglycineamidine synthetase activity Relationships: is a type of GO:0016884